protein localization to early endosome [GO:1902946] (biological process) Definition: A process in which a protein is transported to, or maintained in, a location within an early endosome. References: PMID:22621900 Sources: GOC:TermGenie, GOC:sjp, GO_REF:0000087 Relationships: is a type of protein localization to endosome [GO:0036010] Also known as: protein localisation in early endosome, protein localisation to early endosome, protein localization in early endosome Regulation: regulated by regulation of protein localization to early endosome [GO:1902965]; positively regulated by positive regulation of protein localization to early endosome [GO:1902966]